{
  "term_label": "diadenosine pentaphosphate catabolic process",
  "gene_name": "Diphosphoinositol polyphosphate phosphohydrolase 3-beta",
  "term_id": "GO:1901907",
  "gene_symbol": "NUDT11",
  "gene": "UniProtKB:Q96G61"
}